{
  "term_label": "Unknown molecular function",
  "gene_symbol": "LAPTM4B",
  "term_id": "UNKNOWN:0001",
  "gene_name": "Lysosomal-associated transmembrane protein 4B",
  "gene": "UniProtKB:Q86VI4"
}